{
  "term_label": "Unknown molecular function",
  "term_id": "UNKNOWN:0001",
  "gene": "UniProtKB:Q9P1Y6",
  "gene_name": "PHD and RING finger domain-containing protein 1",
  "gene_symbol": "PHRF1"
}